{
  "term_id": "GO:0000977",
  "term_label": "RNA polymerase II transcription regulatory region sequence-specific DNA binding",
  "gene_name": "Putative zinc finger protein 705G",
  "gene_symbol": "ZNF705G",
  "gene": "UniProtKB:A8MUZ8"
}